{
  "term_label": "DNA-binding transcription factor activity, RNA polymerase II-specific",
  "gene_symbol": "ZNF334",
  "gene": "UniProtKB:Q9HCZ1",
  "term_id": "GO:0000981",
  "gene_name": "Zinc finger protein 334"
}